{
  "gene_name": "Neutral ceramidase",
  "term_id": "GO:0046514",
  "gene": "UniProtKB:Q9NR71",
  "gene_symbol": "ASAH2",
  "term_label": "ceramide catabolic process"
}